{
  "gene": "UniProtKB:Q96PD7",
  "term_id": "GO:0019432",
  "gene_symbol": "DGAT2",
  "term_label": "triglyceride biosynthetic process",
  "gene_name": "Diacylglycerol O-acyltransferase 2"
}